{
  "term_id": "GO:0032456",
  "gene_symbol": "WIPF3",
  "term_label": "endocytic recycling",
  "gene_name": "WAS_WASL-interacting protein family member 3",
  "gene": "UniProtKB:A6NGB9"
}